{
  "gene_symbol": "EPCAM",
  "gene_name": "Epithelial cell adhesion molecule",
  "term_id": "GO:0098641",
  "gene": "UniProtKB:P16422",
  "term_label": "cadherin binding involved in cell-cell adhesion"
}